{
  "gene_symbol": "CEP78",
  "gene": "UniProtKB:Q5JTW2",
  "gene_name": "Centrosomal protein of 78 kDa",
  "term_label": "centrosome",
  "term_id": "GO:0005813"
}